{
  "term_id": "GO:0061630",
  "term_label": "ubiquitin protein ligase activity",
  "gene_name": "E3 ubiquitin-protein ligase RNF186",
  "gene": "UniProtKB:Q9NXI6",
  "gene_symbol": "RNF186"
}